cytokinesis, division site positioning [GO:0007105] (biological process) Relationships: is a type of GO:0032506 Also known as: cytokinesis, site selection, division plane positioning, site selection involved in cell cycle cytokinesis, site selection involved in cytokinesis, contractile ring localization Definition: The process in which a contractile ring is positioned in a specific location. This process is critical for both for both symmetric and asymmetric cell divisions. Regulation: regulated by regulation of cytokinesis, site selection [GO:2000073]; negatively regulated by negative regulation of cytokinesis, site selection [GO:2000075]; positively regulated by positive regulation of cytokinesis, site selection [GO:2000076] References: PMID:26553932, PMID:28162898 Subtypes: GO:1902408